{
  "term_label": "canonical Wnt signaling pathway",
  "gene_name": "Frizzled-5",
  "term_id": "GO:0060070",
  "gene": "UniProtKB:Q13467",
  "gene_symbol": "FZD5"
}